{
  "term_label": "ATP hydrolysis activity",
  "term_id": "GO:0016887",
  "gene_symbol": "ATAD2B",
  "gene": "UniProtKB:Q9ULI0",
  "gene_name": "ATPase family AAA domain-containing protein 2B"
}